podocyte development [GO:0072015] (biological process) Also known as: glomerular visceral epithelial cell development Subtypes: mesonephric podocyte development [GO:0061257], metanephric podocyte development [GO:0072249] Relationships: is_a glomerular epithelial cell development [GO:0072310]; is part of podocyte differentiation [GO:0072112] Definition: The process whose specific outcome is the progression of a glomerular visceral epithelial cell over time, from its formation to the mature structure. A glomerular visceral epithelial cell is a specialized epithelial cell that contains 'feet' that interdigitate with the 'feet' of other glomerular epithelial cells. Sources: GOC:mtg_kidney_jan10